RNA polymerase II cis-regulatory region sequence-specific DNA binding, bending [GO:0044377] (molecular function) Relationships: is a type of RNA polymerase II cis-regulatory region sequence-specific DNA binding [GO:0000978]; is a type of sequence-specific DNA binding, bending [GO:0044374] Definition: Binding to a specific upstream regulatory DNA sequence (transcription factor recognition sequence or binding site) located in cis relative to the transcription start site (i.e., on the same strand of DNA) of a gene transcribed by RNA polymerase II, and distorting the original structure of DNA, typically a straight helix, into a bend, or increasing the bend if the original structure was intrinsically bent due to its sequence. Also known as: RNA polymerase II core promoter proximal region sequence-specific DNA binding, bending, RNA polymerase II promoter proximal region sequence-specific DNA binding, bending, RNA polymerase II proximal promoter region sequence-specific DNA binding, bending, RNA polymerase II proximal promoter sequence-specific DNA binding, bending Sources: GOC:jl, GOC:pg